{
  "term_id": "UNKNOWN:0003",
  "gene_symbol": "TAX1BP1",
  "term_label": "Unknown cellular component",
  "gene": "UniProtKB:Q86VP1",
  "gene_name": "Tax1-binding protein 1"
}